{
  "gene_name": "Max dimerization protein 1",
  "term_label": "DNA-binding transcription factor activity, RNA polymerase II-specific",
  "gene_symbol": "MXD1",
  "term_id": "GO:0000981",
  "gene": "UniProtKB:Q05195"
}